{
  "gene_symbol": "ALKBH3",
  "gene_name": "Alpha-ketoglutarate-dependent dioxygenase alkB homolog 3",
  "gene": "UniProtKB:Q96Q83",
  "term_id": "GO:0005654",
  "term_label": "nucleoplasm"
}